neutrophil extracellular trap formation [GO:0140645] (biological process) Also known as: NET formation Definition: The aggregation, arrangement and bonding together of a set of components to form a neutrophil extracellular trap, a network of extracellular fibers primarily composed of DNA from neutrophils, which bind and neutralizes pathogens. Relationships: is a type of cellular component assembly [GO:0022607] References: PMID:28267716